photosynthesis, light reaction [GO:0019684] (biological process) Definition: The light reactions of photosynthesis, which take place in photosystems II and I. Light energy is harvested and used to power the transfer of electrons among a series of electron donors and acceptors. The final electron acceptor is NADP+, which is reduced to NADPH. NADPH generated from light reactions is used in sugar synthesis in dark reactions. Light reactions also generate a proton motive force across the thylakoid membrane, and the proton gradient is used to synthesize ATP. There are two chemical reactions involved in the light reactions: water oxidation in photosystem II, and NADP reduction in photosystem I. References: PMID:15746074 Regulation: regulated by GO:0042548; negatively regulated by GO:0043155 Also known as: photolysis Relationships: is_a GO:0006091; is part of photosynthesis [GO:0015979]